{
  "gene_name": "Actin-related protein 10",
  "term_id": "GO:0005634",
  "gene_symbol": "ACTR10",
  "gene": "UniProtKB:Q9NZ32",
  "term_label": "nucleus"
}